{
  "term_id": "GO:0005634",
  "gene_name": "Coiled-coil-helix-coiled-coil-helix domain-containing protein 2",
  "gene_symbol": "CHCHD2",
  "term_label": "nucleus",
  "gene": "UniProtKB:Q9Y6H1"
}